{
  "gene_name": "U6 snRNA-associated Sm-like protein LSm8",
  "gene_symbol": "LSM8",
  "term_label": "precatalytic spliceosome",
  "gene": "UniProtKB:O95777",
  "term_id": "GO:0071011"
}